{
  "gene": "UniProtKB:Q96QE2",
  "term_label": "myo-inositol:proton symporter activity",
  "gene_symbol": "SLC2A13",
  "term_id": "GO:0005366",
  "gene_name": "Proton myo-inositol cotransporter"
}